{
  "term_label": "axonogenesis",
  "gene": "UniProtKB:P61371",
  "gene_symbol": "ISL1",
  "gene_name": "Insulin gene enhancer protein ISL-1",
  "term_id": "GO:0007409"
}